{
  "gene_symbol": "TBX18",
  "gene": "UniProtKB:O95935",
  "term_id": "GO:0016331",
  "term_label": "morphogenesis of embryonic epithelium",
  "gene_name": "T-box transcription factor TBX18"
}